{
  "gene_symbol": "LRPAP1",
  "gene": "UniProtKB:P30533",
  "gene_name": "Alpha-2-macroglobulin receptor-associated protein",
  "term_id": "GO:0070326",
  "term_label": "very-low-density lipoprotein particle receptor binding"
}